{
  "gene": "UniProtKB:O75116",
  "gene_name": "Rho-associated protein kinase 2",
  "gene_symbol": "ROCK2",
  "term_id": "GO:0031032",
  "term_label": "actomyosin structure organization"
}